positive regulation of animal organ morphogenesis [GO:0110110] (BP) Definition: Any process that activates or increases the frequency, rate or extent of animal organ morphogenesis. Subtypes: organ induction [GO:0001759], positive regulation of odontogenesis [GO:0042482], GO:0060639, renal vesicle induction [GO:0072034], positive regulation of ureteric bud formation [GO:0072107], positive regulation of nematode pharynx morphogenesis [GO:0110043], GO:1901321, positive regulation of otic vesicle morphogenesis [GO:1904120] Relationships: is a type of positive regulation of developmental process [GO:0051094]; is a type of positive regulation of multicellular organismal process [GO:0051240]; is a type of regulation of animal organ morphogenesis [GO:2000027]; positively regulates animal organ morphogenesis [GO:0009887] Sources: GOC:kmv